{
  "gene": "UniProtKB:A6NL08",
  "gene_name": "Olfactory receptor 6C75",
  "term_id": "GO:0005886",
  "term_label": "plasma membrane",
  "gene_symbol": "OR6C75"
}